alternative respiration [GO:0010230] (biological process) Relationships: is a type of aerobic respiration [GO:0009060] Sources: ISBN:0943088399 Definition: Alternative respiration pathway consumes oxygen, oxidizes NADH to NAD+ and generates water. During electron flow, proton motive force is diminished resulting in fewer molecules of ATP compared to cytochrome pathway. The pathway is found in plants, algae and some protozoa.